{
  "gene_name": "Putative zinc finger protein 876",
  "gene_symbol": "ZNF876P",
  "gene": "UniProtKB:Q49A33",
  "term_label": "DNA-binding transcription factor activity, RNA polymerase II-specific",
  "term_id": "GO:0000981"
}